{
  "term_id": "GO:0055037",
  "gene_name": "RAB11-binding protein RELCH",
  "term_label": "recycling endosome",
  "gene_symbol": "RELCH",
  "gene": "UniProtKB:Q9P260"
}